{
  "gene": "UniProtKB:Q9H2G4",
  "gene_name": "Testis-specific Y-encoded-like protein 2",
  "term_id": "GO:0005634",
  "term_label": "nucleus",
  "gene_symbol": "TSPYL2"
}